{
  "gene_symbol": "CCL3",
  "gene_name": "C-C motif chemokine 3",
  "gene": "UniProtKB:P10147",
  "term_id": "GO:0061844",
  "term_label": "antimicrobial humoral immune response mediated by antimicrobial peptide"
}